positive regulation of single stranded viral RNA replication via double stranded DNA intermediate [GO:0045870] (biological process) Sources: GOC:go_curators Also known as: positive regulation of retroviral genome replication, up regulation of retroviral genome replication, up-regulation of retroviral genome replication, upregulation of retroviral genome replication, activation of retroviral genome replication, stimulation of retroviral genome replication Definition: Any process that activates or increases the frequency, rate or extent of retroviral genome replication. Relationships: is a type of positive regulation of viral genome replication [GO:0045070]; is a type of regulation of single stranded viral RNA replication via double stranded DNA intermediate [GO:0045091]; is a type of positive regulation of RNA biosynthetic process [GO:1902680]; positively regulates single stranded viral RNA replication via double stranded DNA intermediate [GO:0039692]